{
  "term_id": "UNKNOWN:0003",
  "term_label": "Unknown cellular component",
  "gene": "UniProtKB:Q9GZX5",
  "gene_name": "Zinc finger protein 350",
  "gene_symbol": "ZNF350"
}